{
  "gene": "UniProtKB:P08574",
  "gene_name": "Cytochrome c1, heme protein, mitochondrial",
  "gene_symbol": "CYC1",
  "term_label": "mitochondrial electron transport, ubiquinol to cytochrome c",
  "term_id": "GO:0006122"
}